negative regulation of brood size [GO:0090728] (biological process) Definition: Any process that decreases brood size. Brood size is the number of progeny that survive embryogenesis and are cared for at one time. Sources: GOC:rz Relationships: is a type of biological regulation [GO:0065007]